{
  "term_label": "signal transduction",
  "term_id": "GO:0007165",
  "gene": "UniProtKB:Q15612",
  "gene_name": "Olfactory receptor 1Q1",
  "gene_symbol": "OR1Q1"
}